{
  "term_id": "GO:0045292",
  "gene_symbol": "SF1",
  "gene_name": "Splicing factor 1",
  "term_label": "mRNA cis splicing, via spliceosome",
  "gene": "UniProtKB:Q15637"
}